{
  "gene": "UniProtKB:P0DW14",
  "term_id": "GO:0051123",
  "gene_name": "TATA-box-binding protein-associated factor 11-like protein 10",
  "gene_symbol": "TAF11L10",
  "term_label": "RNA polymerase II preinitiation complex assembly"
}